{
  "term_label": "RNA polymerase II general transcription initiation factor activity",
  "term_id": "GO:0016251",
  "gene": "UniProtKB:A0A1W2PRV1",
  "gene_symbol": "TAF11L3",
  "gene_name": "TATA-box-binding protein-associated factor 11-like protein 3"
}